C-terminal protein amino acid modification [GO:0018410] (biological process) Subtypes: C-terminal protein methylation [GO:0006481], C-terminal protein lipidation [GO:0006501], C-terminal protein deglutamylation [GO:0035609] Sources: GOC:mah Definition: The alteration of the C-terminal amino acid residue in a protein. Relationships: is a type of post-translational protein modification [GO:0043687] Also known as: peptide or protein carboxyl-terminal blocking, peptide/protein carboxyl-terminal blocking